{
  "gene_symbol": "UPK3B",
  "gene": "UniProtKB:Q9BT76",
  "term_id": "UNKNOWN:0002",
  "gene_name": "Uroplakin-3b",
  "term_label": "Unknown biological process"
}